{
  "gene": "UniProtKB:O75368",
  "gene_symbol": "SH3BGRL",
  "gene_name": "Adapter SH3BGRL",
  "term_label": "proteasome-mediated ubiquitin-dependent protein catabolic process",
  "term_id": "GO:0043161"
}